{
  "term_id": "GO:0030855",
  "gene": "UniProtKB:P13646",
  "gene_name": "Keratin, type I cytoskeletal 13",
  "gene_symbol": "KRT13",
  "term_label": "epithelial cell differentiation"
}